cellular response to oscillatory fluid shear stress [GO:0097704] (biological process) Relationships: is_a GO:0071498; is a type of response to oscillatory fluid shear stress [GO:0097702] References: PMID:21768538 Sources: GOC:BHF, GOC:BHF_miRNA, GOC:bc Definition: Any response to oscillatory fluid shear stress that occurs at the level of a cell. Subtypes: GO:0097706